{
  "term_id": "GO:0044325",
  "gene": "UniProtKB:A0A1B0GVM2",
  "gene_symbol": "TCAF2C",
  "term_label": "transmembrane transporter binding",
  "gene_name": "TRPM8 channel associated factor 2C (Fragment)"
}